{
  "gene_symbol": "ZNF648",
  "term_label": "DNA-binding transcription factor activity, RNA polymerase II-specific",
  "gene": "UniProtKB:Q5T619",
  "gene_name": "Zinc finger protein 648",
  "term_id": "GO:0000981"
}